{
  "term_id": "GO:0001669",
  "gene_name": "Semenogelin-2",
  "gene": "UniProtKB:Q02383",
  "gene_symbol": "SEMG2",
  "term_label": "acrosomal vesicle"
}